{
  "gene_symbol": "ZNF789",
  "gene": "UniProtKB:Q5FWF6",
  "term_label": "DNA-binding transcription factor activity, RNA polymerase II-specific",
  "gene_name": "Zinc finger protein 789",
  "term_id": "GO:0000981"
}